{
  "gene_name": "RNA-binding motif protein, X chromosome",
  "gene_symbol": "RBMX",
  "gene": "UniProtKB:P38159",
  "term_label": "mRNA splicing, via spliceosome",
  "term_id": "GO:0000398"
}